{
  "gene_name": "ETS-related transcription factor Elf-4",
  "term_label": "cell differentiation",
  "gene_symbol": "ELF4",
  "term_id": "GO:0030154",
  "gene": "UniProtKB:Q99607"
}